{
  "gene_symbol": "MCRIP2",
  "gene_name": "MAPK regulated corepressor interacting protein 2",
  "gene": "UniProtKB:Q9BUT9",
  "term_label": "Unknown cellular component",
  "term_id": "UNKNOWN:0003"
}